inositol-1,4,5-trisphosphate 3-kinase activity [GO:0008440] (molecular function) Sources: RHEA:11020 Definition: Catalysis of the reaction: 1D-myo-inositol 1,4,5-trisphosphate + ATP = 1D-myo-inositol 1,3,4,5-tetrakisphosphate + ADP + H+. Relationships: is a type of inositol trisphosphate kinase activity [GO:0051766] Also known as: 1D-myo-inositol-trisphosphate 3-kinase activity, inositol trisphosphate 3-kinase activity, inositol-trisphosphate 3-kinase activity, IP3 3-kinase activity, IP3K activity, Ins(1,4,5)P3 3-kinase activity